{
  "term_id": "GO:0005886",
  "gene_name": "Immunoglobulin subtype domain-containing protein",
  "gene_symbol": "A0A1W2PRS3",
  "gene": "UniProtKB:A0A1W2PRS3",
  "term_label": "plasma membrane"
}